UDP-4-amino-4-deoxy-L-arabinose formyltransferase activity [GO:0099619] (molecular function) Also known as: 10-formyltetrahydrofolate:UDP-4-amino-4-deoxy-beta-L-arabinose N-formyltransferase activity, ArnAFT activity, UDP-L-Ara4N formyltransferase activity References: PMID:15695810, PMID:15807526, PMID:15809294, PMID:15939024, PMID:17928292 Definition: Catalysis of the reaction: 10-formyltetrahydrofolate + UDP-4-amino-4-deoxy-beta-L-arabinopyranose = 5,6,7,8-tetrahydrofolate + UDP-4-deoxy-4-formamido-beta-L-arabinopyranose. Relationships: is a type of hydroxymethyl-, formyl- and related transferase activity [GO:0016742]